MHC class II protein complex binding [GO:0023026] (molecular function) Sources: GOC:mtg_signal, GOC:vw Definition: Binding to a class II major histocompatibility complex. Relationships: is a type of MHC protein complex binding [GO:0023023]